{
  "term_label": "regulation of the force of skeletal muscle contraction",
  "term_id": "GO:0014728",
  "gene_symbol": "KBTBD13",
  "gene_name": "Kelch repeat and BTB domain-containing protein 13",
  "gene": "UniProtKB:C9JR72"
}